{
  "gene": "UniProtKB:P20815",
  "gene_symbol": "CYP3A5",
  "term_id": "GO:0008202",
  "term_label": "steroid metabolic process",
  "gene_name": "Cytochrome P450 3A5"
}